{
  "gene_symbol": "VPS41",
  "term_id": "GO:0009267",
  "gene": "UniProtKB:P49754",
  "gene_name": "Vacuolar protein sorting-associated protein 41 homolog",
  "term_label": "cellular response to starvation"
}